{
  "term_label": "cell surface",
  "gene_name": "Syndecan-1",
  "gene": "UniProtKB:P18827",
  "term_id": "GO:0009986",
  "gene_symbol": "SDC1"
}